{
  "gene": "UniProtKB:Q14565",
  "gene_name": "Meiotic recombination protein DMC1_LIM15 homolog",
  "term_label": "single-stranded DNA binding",
  "term_id": "GO:0003697",
  "gene_symbol": "DMC1"
}